methylenetetrahydrofolate dehydrogenase (NADP+) activity [GO:0004488] (molecular function) Relationships: is a type of oxidoreductase activity, acting on the CH-NH group of donors, NAD or NADP as acceptor [GO:0016646] Sources: EC:1.5.1.5, RHEA:22812 Definition: Catalysis of the reaction: 5,10-methylenetetrahydrofolate + NADP+ = 5,10-methenyltetrahydrofolate + NADPH. Also known as: 5,10-methylenetetrahydrofolate:NADP oxidoreductase activity, 5,10-methylenetetrahydrofolate:NADP+ oxidoreductase activity